{
  "gene_name": "Zinc finger protein 692",
  "gene": "UniProtKB:Q9BU19",
  "term_id": "GO:0006357",
  "term_label": "regulation of transcription by RNA polymerase II",
  "gene_symbol": "ZNF692"
}